positive regulation of store-operated calcium entry [GO:0106129] (biological process) Relationships: is a type of positive regulation of calcium ion transport [GO:0051928]; is a type of regulation of store-operated calcium entry [GO:2001256]; positively regulates GO:0002115 References: PMID:23447642 Sources: GOC:BHF, GOC:BHF_miRNA, GOC:rph Definition: Any process that activates or increases the frequency, rate or extent of store-operated calcium entry.